protein denucleotidylation [GO:0044601] (biological process) Subtypes: GO:0044602 References: PMID:21734656 Sources: GOC:sp Relationships: is_a protein modification process [GO:0036211] Definition: The removal of a nucleotide from a protein amino acid.